observational learning [GO:0098597] (BP) Note: Observation here is used in a broad sense to include perception of the behavior of others via any form or combination of forms of sensory perception (visual, auditory etc). Observational learning is broader than imitative learning in that it does not require a duplication of the behavior exhibited by the model. Relationships: is a type of learning [GO:0007612] Subtypes: imitative learning [GO:0098596] Definition: Learning that occurs through observing the behavior of others. Sources: GOC:dos, Wikipedia:Observational_learning&oldid=603524137